apigenin 7-O-methyltransferase activity [GO:0102529] (molecular function) Relationships: is a type of GO:0008168 Definition: Catalysis of the reaction: apigenin + S-adenosyl-L-methionine = genkwanin + H+ + S-adenosyl-L-homocysteine. Sources: RHEA:73071